{
  "gene_symbol": "SLC8B1",
  "gene_name": "Mitochondrial sodium_calcium exchanger protein",
  "term_label": "calcium:sodium antiporter activity",
  "term_id": "GO:0005432",
  "gene": "UniProtKB:Q6J4K2"
}